{
  "term_label": "Unknown molecular function",
  "gene_symbol": "ALDH7A1",
  "gene": "UniProtKB:P49419",
  "term_id": "UNKNOWN:0001",
  "gene_name": "Alpha-aminoadipic semialdehyde dehydrogenase"
}